glutamate-putrescine ligase activity [GO:0034024] (molecular function) Definition: Catalysis of the reaction: L-glutamate + ATP + putrescine = gamma-L-glutamylputrescine + ADP + 2 H+ + phosphate. Sources: EC:6.3.1.11, RHEA:13633 Also known as: L-glutamate:putrescine ligase (ADP-forming) activity, YcjK, gamma-glutamylputrescine synthetase activity Relationships: is a type of acid-ammonia (or amide) ligase activity [GO:0016880]